{
  "gene_symbol": "SLC6A8",
  "gene": "UniProtKB:P48029",
  "term_label": "plasma membrane",
  "term_id": "GO:0005886",
  "gene_name": "Sodium- and chloride-dependent creatine transporter 1"
}